{
  "gene_name": "Nuclear mitotic apparatus protein 1",
  "term_id": "GO:0005876",
  "gene_symbol": "NUMA1",
  "term_label": "spindle microtubule",
  "gene": "UniProtKB:Q14980"
}